{
  "term_label": "neuron projection",
  "gene_symbol": "RGS9BP",
  "gene": "UniProtKB:Q6ZS82",
  "gene_name": "Regulator of G-protein signaling 9-binding protein",
  "term_id": "GO:0043005"
}